{
  "term_label": "polyadenylation-dependent ncRNA catabolic process",
  "gene_symbol": "TENT4A",
  "gene": "UniProtKB:Q5XG87",
  "gene_name": "Terminal nucleotidyltransferase 4A",
  "term_id": "GO:0043634"
}